{
  "gene": "UniProtKB:Q8WWF3",
  "gene_symbol": "SSMEM1",
  "term_label": "Unknown molecular function",
  "gene_name": "Serine-rich single-pass membrane protein 1",
  "term_id": "UNKNOWN:0001"
}